{
  "gene_name": "Zinc finger FYVE domain-containing protein 16",
  "term_label": "endosomal transport",
  "gene_symbol": "ZFYVE16",
  "term_id": "GO:0016197",
  "gene": "UniProtKB:Q7Z3T8"
}